{
  "gene_name": "Protein-glutamine gamma-glutamyltransferase 2",
  "gene_symbol": "TGM2",
  "term_id": "GO:0051561",
  "gene": "UniProtKB:P21980",
  "term_label": "positive regulation of mitochondrial calcium ion concentration"
}